{
  "gene_name": "E3 ubiquitin-protein ligase Topors",
  "gene": "UniProtKB:Q9NS56",
  "term_id": "GO:0016607",
  "gene_symbol": "TOPORS",
  "term_label": "nuclear speck"
}